{
  "gene_name": "RNA-binding protein FXR2",
  "gene_symbol": "FXR2",
  "term_label": "neuron projection",
  "term_id": "GO:0043005",
  "gene": "UniProtKB:P51116"
}